{
  "gene_name": "Protein Wnt-2",
  "term_label": "cell fate commitment",
  "gene": "UniProtKB:P09544",
  "gene_symbol": "WNT2",
  "term_id": "GO:0045165"
}